karyomere membrane fusion [GO:0061472] (biological process) Relationships: is a type of organelle membrane fusion [GO:0090174]; is_a GO:1903047; is part of mitotic nuclear membrane reassembly [GO:0007084] References: PMID:2734396 Sources: GOC:dph Definition: Process whereby karyomere membranes fuse during interphase to form a single lobed nucleus.